{
  "term_label": "fatty-acyl-CoA synthase activity",
  "gene_symbol": "ACSM3",
  "gene": "UniProtKB:Q53FZ2",
  "gene_name": "Acyl-coenzyme A synthetase ACSM3, mitochondrial",
  "term_id": "GO:0004321"
}